{
  "gene_name": "Splicing factor 3B subunit 1",
  "gene": "UniProtKB:O75533",
  "gene_symbol": "SF3B1",
  "term_id": "GO:0071013",
  "term_label": "catalytic step 2 spliceosome"
}